{
  "term_id": "UNKNOWN:0001",
  "gene_symbol": "IGKV1-33",
  "gene": "UniProtKB:P01594",
  "term_label": "Unknown molecular function",
  "gene_name": "Immunoglobulin kappa variable 1-33"
}